positive regulation of antigen processing and presentation of lipid antigen via MHC class Ib [GO:0002600] (biological process) Relationships: is a type of positive regulation of antigen processing and presentation via MHC class Ib [GO:0002594]; is a type of regulation of antigen processing and presentation of lipid antigen via MHC class Ib [GO:0002598]; positively regulates GO:0048003 Definition: Any process that activates or increases the frequency, rate, or extent of antigen processing and presentation of lipid antigen via MHC class Ib. Also known as: positive regulation of lipid antigen processing and presentation via MHC class Ib, up regulation of antigen processing and presentation of lipid antigen via MHC class Ib, up-regulation of antigen processing and presentation of lipid antigen via MHC class Ib, upregulation of antigen processing and presentation of lipid antigen via MHC class Ib, activation of antigen processing and presentation of lipid antigen via MHC class Ib, stimulation of antigen processing and presentation of lipid antigen via MHC class Ib Sources: GOC:add